{
  "gene_name": "Adaptin ear-binding coat-associated protein 1",
  "gene": "UniProtKB:Q8NC96",
  "term_id": "GO:0030125",
  "term_label": "clathrin vesicle coat",
  "gene_symbol": "NECAP1"
}